9-cis-10'-apo-beta-carotenal cleavage oxygenase activity [GO:0102396] (molecular function) Sources: EC:1.13.11.69, GOC:pz Definition: Catalysis of the reaction: 9-cis-10'-apo-beta-carotenal + 2 O2 = carlactone + (2E,4E,6E)-7-hydroxy-4-methylhepta-2,4,6-trienal. Relationships: is a type of oxidoreductase activity, acting on single donors with incorporation of molecular oxygen, incorporation of two atoms of oxygen [GO:0016702]